{
  "gene_symbol": "TMEM127",
  "gene": "UniProtKB:O75204",
  "gene_name": "Transmembrane protein 127",
  "term_id": "UNKNOWN:0001",
  "term_label": "Unknown molecular function"
}